{
  "term_label": "immune receptor activity",
  "gene": "UniProtKB:Q6GTX8",
  "term_id": "GO:0140375",
  "gene_name": "Leukocyte-associated immunoglobulin-like receptor 1",
  "gene_symbol": "LAIR1"
}